protein localization to cell division site involved in cytokinesis, actomyosin contractile ring assembly [GO:1902575] (biological process) References: PMID:24127216 Sources: GOC:TermGenie, GOC:al Subtypes: protein localization to cell division site involved in mitotic actomyosin contractile ring assembly [GO:1903476] Relationships: is a type of protein localization to cell division site [GO:0072741]; is part of actomyosin contractile ring assembly [GO:0000915] Definition: Any protein localization to cell division site that is involved in cytokinesis, actomyosin contractile ring assembly. Also known as: protein localisation to cell division site involved in contractile ring assembly, protein localisation to cell division site involved in cytokinesis, actomyosin contractile ring assembly, protein localization to cell division site involved in contractile ring assembly, protein localisation to cell division site involved in constriction ring assembly, protein localization to cell division site involved in constriction ring assembly, protein localisation to cell division site involved in cytokinesis, actomyosin contractile ring formation, protein localisation to cell division site involved in cytokinesis, actomyosin ring biosynthesis, protein localisation to cell division site involved in cytokinesis, actomyosin ring formation, protein localisation to cell division site involved in cytokinesis, contractile ring assembly, protein localization to cell division site involved in cytokinesis, actomyosin contractile ring formation, protein localization to cell division site involved in cytokinesis, actomyosin ring biosynthesis, protein localization to cell division site involved in cytokinesis, actomyosin ring formation, protein localization to cell division site involved in cytokinesis, contractile ring assembly